LEM domain binding [GO:0097726] (molecular function) Also known as: LAP2, emerin, MAN1 domain binding, lamina-associated polypeptide, emerin, MAN1 domain binding References: PMID:22399800 Sources: GOC:rz, InterPro:IPR003887 Definition: Binding to a LEM domain. The LEM domain (for lamina-associated polypeptide, emerin, MAN1 domain) is present in a group of nuclear proteins that bind chromatin through interaction of the LEM motif with the conserved DNA crosslinking protein, barrier-to-autointegration factor (BAF). Relationships: is a type of protein domain specific binding [GO:0019904]